{
  "term_id": "GO:0005813",
  "gene": "UniProtKB:Q9UJC3",
  "gene_symbol": "HOOK1",
  "term_label": "centrosome",
  "gene_name": "Protein Hook homolog 1"
}